{
  "gene": "UniProtKB:Q8N2K0",
  "gene_symbol": "ABHD12",
  "term_label": "phosphatidylserine catabolic process",
  "gene_name": "Lysophosphatidylserine lipase ABHD12",
  "term_id": "GO:0006660"
}